{
  "gene_name": "Iroquois-class homeodomain protein IRX-5",
  "gene_symbol": "IRX5",
  "term_id": "GO:0000978",
  "term_label": "RNA polymerase II cis-regulatory region sequence-specific DNA binding",
  "gene": "UniProtKB:P78411"
}